{
  "term_id": "GO:0005634",
  "term_label": "nucleus",
  "gene_symbol": "TRMT1L",
  "gene_name": "TRMT1-like protein",
  "gene": "UniProtKB:Q7Z2T5"
}